{
  "gene_name": "V(D)J recombination-activating protein 1",
  "term_label": "nucleus",
  "gene": "UniProtKB:P15918",
  "term_id": "GO:0005634",
  "gene_symbol": "RAG1"
}